oogonium development [GO:0075263] (biological process) Definition: The process that leads to the development of an oogonium, a female gametangium of Oomycetes, containing one or more gametes. Sources: GOC:pamgo_curators Relationships: is a type of spore-bearing structure development [GO:0075259] Regulation: regulated by regulation of oogonium development [GO:0075264]; positively regulated by GO:0075265; negatively regulated by negative regulation of oogonium development [GO:0075266]